{
  "gene_symbol": "SUPT16H",
  "gene": "UniProtKB:Q9Y5B9",
  "term_id": "GO:0006337",
  "term_label": "nucleosome disassembly",
  "gene_name": "FACT complex subunit SPT16"
}